positive regulation of DNA catabolic process [GO:1903626] (biological process) Definition: Any process that activates or increases the frequency, rate or extent of DNA catabolic process. Relationships: is_a positive regulation of catabolic process [GO:0009896]; is a type of positive regulation of DNA metabolic process [GO:0051054]; is a type of regulation of DNA catabolic process [GO:1903624]; RO_0002213 GO:0006308 Also known as: positive regulation of DNA breakdown, positive regulation of DNA catabolism, positive regulation of DNA degradation, up regulation of DNA breakdown, up regulation of DNA catabolic process, up regulation of DNA catabolism, up regulation of DNA degradation, up-regulation of DNA breakdown, up-regulation of DNA catabolic process, up-regulation of DNA catabolism, up-regulation of DNA degradation, upregulation of DNA breakdown, upregulation of DNA catabolic process, upregulation of DNA catabolism, upregulation of DNA degradation, activation of DNA breakdown, activation of DNA catabolic process, activation of DNA catabolism, activation of DNA degradation Subtypes: GO:1902512 References: PMID:2001740 Sources: GOC:TermGenie, GO_REF:0000058